intracellular abscisic acid homeostasis [GO:1902266] (biological process) Definition: A homeostatic process involved in the maintenance of a steady state level of abscisic acid within a cell. References: PMID:23252460 Sources: GOC:TermGenie Relationships: is a type of intracellular chemical homeostasis [GO:0055082]; is a type of abscisic acid homeostasis [GO:1902265] Also known as: cellular 2-cis-abscisate homeostasis, cellular ABA homeostasis